cell proliferation in bone marrow [GO:0071838] (biological process) Definition: The multiplication or reproduction of cells, resulting in the expansion of a cell population in the bone marrow. References: PMID:17063141 Sources: GOC:mah, GOC:yaf Also known as: bone marrow cell proliferation Relationships: is a type of cell population proliferation [GO:0008283] Regulation: regulated by regulation of cell proliferation in bone marrow [GO:0071863]; positively regulated by positive regulation of cell proliferation in bone marrow [GO:0071864]; negatively regulated by negative regulation of cell proliferation in bone marrow [GO:1903769]